UDP-N-acetylmuramoyl-L-alanyl-D-glutamate-L-lysine ligase activity [GO:0047482] (molecular function) Definition: Catalysis of the reaction: L-lysine + ATP + UDP-N-acetylmuramoyl-L-alanyl-D-glutamate = ADP + 2 H+ + phosphate + UDP-N-acetylmuramoyl-L-alanyl-D-glutamyl-L-lysine. Relationships: is a type of acid-amino acid ligase activity [GO:0016881] Sources: EC:6.3.2.7, RHEA:17969 Also known as: L-lysine-adding enzyme activity, MurE synthetase activity, UDP-N-acetylmuramoyl-L-alanyl-D-glutamate:L-lysine gamma-ligase (ADP-forming), UDP-N-acetylmuramoyl-L-alanyl-D-glutamyl-L-lysine synthetase activity, UPD-MurNAc-L-Ala-D-Glu:L-Lys ligase activity, uridine diphospho-N-acetylmuramoylalanyl-D-glutamyllysine synthetase activity